T=27/pseudo27 icosahedral capsid [GO:0160170] (cellular component) Relationships: is a type of icosahedral viral capsid [GO:0019030] Definition: The protein coat that surrounds the infective nucleic acid in some virus particles where the subunits (capsomeres) are arranged to form an icosahedron with T=27 or pseudo T=27 symmetry. Sources: VZ:1556